{
  "term_label": "Unknown cellular component",
  "gene": "UniProtKB:A0A0B4J1X8",
  "gene_symbol": "IGHV3-43",
  "term_id": "UNKNOWN:0003",
  "gene_name": "Immunoglobulin heavy variable 3-43"
}